{
  "gene": "UniProtKB:Q13454",
  "gene_symbol": "TUSC3",
  "term_id": "GO:0018279",
  "term_label": "protein N-linked glycosylation via asparagine",
  "gene_name": "Tumor suppressor candidate 3"
}